shikimate 3-dehydrogenase (NAD+) activity [GO:0052734] (molecular function) Also known as: DHS reductase activity, dehydroshikimic reductase activity, shikimate oxidoreductase activity, shikimate:NAD(P)(+) oxidoreductase activity, 3-dehydroshikimate reductase activity, 3-dehydroshikimic reductase activity, shikimate:NAD(P)(+) 3-oxidoreductase activity Sources: RHEA:17741 Definition: Catalysis of the reaction: shikimate + NAD+ = 3-dehydroshikimate + NADH + H+. Relationships: is a type of GO:0016616